{
  "term_label": "establishment of cell polarity",
  "gene_name": "Rho-related GTP-binding protein RhoQ",
  "term_id": "GO:0030010",
  "gene": "UniProtKB:P17081",
  "gene_symbol": "RHOQ"
}